methane monooxygenase [NAD(P)H] activity [GO:0015049] (molecular function) Relationships: is a type of oxidoreductase activity, acting on paired donors, with incorporation or reduction of molecular oxygen, NAD(P)H as one donor, and incorporation of one atom of oxygen [GO:0016709] References: PMID:10896210 Sources: EC:1.14.13.25 Definition: Catalysis of the reaction: methane + NAD(P)H + H+ + O2 = methanol + NAD(P)+ + H2O. Also known as: methane hydroxylase activity, methane,NAD(P)H:oxygen oxidoreductase (hydroxylating)